sesquiterpenoid metabolic process [GO:0006714] (biological process) Definition: The chemical reactions and pathways involving sesquiterpenoid compounds, terpenoids with three isoprene units. Sources: ISBN:0198547684 Also known as: sesquiterpenoid metabolism Relationships: is a type of GO:0006721 Subtypes: juvenile hormone metabolic process [GO:0006716], abscisic acid metabolic process [GO:0009687], GO:0016106, sesquiterpenoid catabolic process [GO:0016107], farnesol metabolic process [GO:0016487], strigolactone metabolic process [GO:1901600]